gastrin-induced gastric acid secretion [GO:0001698] (BP) Sources: GOC:hjd Relationships: is a type of gastric acid secretion [GO:0001696]; has part gastrin receptor activity [GO:0015054] Definition: The regulated release of gastric acid induced by the interaction of gastrin with its receptor. Regulation: regulated by regulation of gastrin-induced gastric acid secretion [GO:1903639]; negatively regulated by negative regulation of gastrin-induced gastric acid secretion [GO:1903640]; positively regulated by GO:1903641